{
  "gene": "UniProtKB:Q76L83",
  "gene_name": "Putative Polycomb group protein ASXL2",
  "term_label": "peroxisome proliferator activated receptor binding",
  "term_id": "GO:0042975",
  "gene_symbol": "ASXL2"
}